{
  "gene_name": "Telomerase reverse transcriptase",
  "term_id": "GO:0042162",
  "term_label": "telomeric DNA binding",
  "gene_symbol": "TERT",
  "gene": "UniProtKB:O14746"
}